{
  "term_id": "UNKNOWN:0001",
  "gene_name": "Syntaxin-18",
  "gene_symbol": "STX18",
  "term_label": "Unknown molecular function",
  "gene": "UniProtKB:Q9P2W9"
}